{
  "term_label": "glycine decarboxylation via glycine cleavage system",
  "gene_symbol": "GLDC",
  "gene": "UniProtKB:P23378",
  "gene_name": "Glycine dehydrogenase (decarboxylating), mitochondrial",
  "term_id": "GO:0019464"
}